{
  "gene_name": "G antigen 12G",
  "term_id": "UNKNOWN:0002",
  "gene_symbol": "GAGE12G",
  "term_label": "Unknown biological process",
  "gene": "UniProtKB:P0CL81"
}